response to activity [GO:0014823] (biological process) Sources: GOC:mtg_muscle Relationships: is a type of response to stimulus [GO:0050896] Definition: Any process that results in a change in state or activity of a cell or an organism (in terms of movement, secretion, enzyme production, gene expression, etc.) as a result of an activity stimulus. Subtypes: response to muscle activity [GO:0014850], detection of activity [GO:0014865] Also known as: response to exercise